cardiac fibroblast cell fate commitment [GO:0060937] (biological process) Relationships: is a type of cardiac cell fate commitment [GO:0060911]; is part of cardiac fibroblast cell differentiation [GO:0060935] Definition: The commitment of cells to a cardiac fibroblast fate and their capacity to differentiate into cardiac fibroblast cells. A cardiac fibroblast is a connective tissue cell in the heart which secretes an extracellular matrix rich in collagen and other macromolecules. Subtypes: GO:0060941, GO:0060944 Sources: GOC:mtg_heart